{
  "term_label": "Unknown cellular component",
  "gene_symbol": "DHRS7",
  "gene": "UniProtKB:Q9Y394",
  "term_id": "UNKNOWN:0003",
  "gene_name": "Dehydrogenase_reductase SDR family member 7"
}